mRNA cleavage and polyadenylation specificity factor complex [GO:0005847] (cellular component) Definition: A multisubunit complex that binds to the canonical AAUAAA hexamer and to U-rich upstream sequence elements on the pre-mRNA, thereby stimulating the otherwise weakly active and nonspecific polymerase to elongate efficiently RNAs containing a poly(A) signal. References: PMID:14749727 Relationships: is a type of GO:0005849 Also known as: CPF complex, CPSF complex, CFII complex, cleavage and polyadenylylation specificity factor activity